peroxisome membrane class-1 targeting sequence binding [GO:0036105] (molecular function) References: PMID:14709540, PMID:17020786 Sources: GOC:pm Note: Currently identified mPTSs vary greatly in length, and cannot be distinguished by primary structure analysis, suggesting that the peroxisomal sorting information is not contained within a specific amino acid sequence. There do however appear to be two classes of mPTSs: class 1 mPTSs that are bound by PEX19 and imported in a PEX19-dependent manner, and class 2 mPTSs that are not bound by PEX19 and mediate protein import independently of PEX19. The two classes cannot be defined based on their amino acid sequence. Relationships: is a type of peroxisome membrane targeting sequence binding [GO:0033328] Definition: Binding to a class I peroxisomal membrane targeting sequence, any of several sequences of amino acids within a protein that can act as a signal for the localization of the protein into the peroxisome membrane in a PEX19-dependent manner. Also known as: class 1 mPTS binding, PEX19-dependent mPTS binding